acetate metabolic process [GO:0006083] (biological process) Definition: The chemical reactions and pathways involving acetate, the anion of acetic acid. Sources: GOC:go_curators Also known as: acetate metabolism Relationships: is_a monocarboxylic acid metabolic process [GO:0032787] Subtypes: methanogenesis, from acetate [GO:0019385], acetate biosynthetic process [GO:0019413], acetyl-CoA biosynthetic process from acetate [GO:0019427], L-lysine fermentation [GO:0019475], L-glutamate catabolic process via 2-hydroxyglutarate [GO:0019552], pyruvate fermentation to acetate [GO:0019654], GO:0019658, GO:0019664, pyruvate biosynthetic process from acetate [GO:0019687], GO:0045122, acetate catabolic process [GO:0045733], GO:0052776